{
  "term_id": "GO:0007186",
  "term_label": "G protein-coupled receptor signaling pathway",
  "gene": "UniProtKB:O00254",
  "gene_name": "Proteinase-activated receptor 3",
  "gene_symbol": "F2RL2"
}